{
  "gene_symbol": "KLK7",
  "gene": "UniProtKB:P49862",
  "term_label": "serine-type endopeptidase activity",
  "term_id": "GO:0004252",
  "gene_name": "Kallikrein-7"
}